{
  "gene_name": "Lysyl oxidase homolog 3",
  "gene_symbol": "LOXL3",
  "term_id": "GO:0030199",
  "term_label": "collagen fibril organization",
  "gene": "UniProtKB:P58215"
}